oxidoreductase activity, acting on the CH-NH group of donors [GO:0016645] (molecular function) Also known as: oxidoreductase activity, acting on the CH-NH group of donors, other acceptors Sources: GOC:ai Subtypes: oxidoreductase activity, acting on the CH-NH group of donors, NAD or NADP as acceptor [GO:0016646], oxidoreductase activity, acting on the CH-NH group of donors, oxygen as acceptor [GO:0016647], oxidoreductase activity, acting on the CH-NH group of donors, disulfide as acceptor [GO:0016648], oxidoreductase activity, acting on the CH-NH group of donors, quinone or similar compound as acceptor [GO:0016649], nicotine dehydrogenase activity [GO:0018535], coenzyme F420-dependent N5,N10-methenyltetrahydromethanopterin reductase activity [GO:0018537], cytokinin dehydrogenase activity [GO:0019139], GO:0030268, oxidoreductase activity, acting on the CH-NH group of donors, iron-sulfur protein as acceptor [GO:0033694], 6-hydroxypseudooxynicotine dehydrogenase activity [GO:0034909], reduced coenzyme F420 dehydrogenase activity [GO:0043738], oxidoreductase activity, acting on the CH-NH group of donors, flavin as acceptor [GO:0046997], L-pipecolate dehydrogenase activity [GO:0050030], methylglutamate dehydrogenase activity [GO:0050099], GO:0050289 Definition: Catalysis of an oxidation-reduction (redox) reaction in which a CH-NH group acts as a hydrogen or electron donor and reduces a hydrogen or electron acceptor. Relationships: is a type of GO:0016491